{
  "term_id": "GO:0016460",
  "term_label": "myosin II complex",
  "gene": "UniProtKB:Q9UKX3",
  "gene_name": "Myosin-13",
  "gene_symbol": "MYH13"
}